{
  "term_label": "synapse assembly",
  "gene": "UniProtKB:Q5T601",
  "gene_symbol": "ADGRF1",
  "term_id": "GO:0007416",
  "gene_name": "Adhesion G-protein coupled receptor F1"
}